{
  "gene_name": "Putative ankyrin repeat domain-containing protein 20A5",
  "gene": "UniProtKB:A0PJZ0",
  "term_label": "Unknown cellular component",
  "gene_symbol": "ANKRD20A5P",
  "term_id": "UNKNOWN:0003"
}